{
  "term_id": "GO:0000981",
  "gene_symbol": "NKX3-2",
  "gene_name": "Homeobox protein Nkx-3.2",
  "gene": "UniProtKB:P78367",
  "term_label": "DNA-binding transcription factor activity, RNA polymerase II-specific"
}